{
  "gene_name": "G-protein coupled receptor 183",
  "gene": "UniProtKB:P32249",
  "gene_symbol": "GPR183",
  "term_id": "GO:0002312",
  "term_label": "B cell activation involved in immune response"
}